{
  "term_id": "GO:0005737",
  "gene_symbol": "ATE1",
  "term_label": "cytoplasm",
  "gene": "UniProtKB:O95260",
  "gene_name": "Arginyl-tRNA--protein transferase 1"
}